{
  "term_id": "GO:0005614",
  "gene_name": "Kazal-type serine protease inhibitor domain-containing protein 1",
  "term_label": "interstitial matrix",
  "gene_symbol": "KAZALD1",
  "gene": "UniProtKB:Q96I82"
}